{
  "gene_name": "Gamma-aminobutyric acid receptor-associated protein-like 1",
  "term_id": "GO:0006995",
  "gene": "UniProtKB:Q9H0R8",
  "gene_symbol": "GABARAPL1",
  "term_label": "cellular response to nitrogen starvation"
}